{
  "term_id": "GO:0005737",
  "gene_symbol": "MAP4K2",
  "gene": "UniProtKB:Q12851",
  "gene_name": "Mitogen-activated protein kinase kinase kinase kinase 2",
  "term_label": "cytoplasm"
}